{
  "gene_name": "Delta-1-pyrroline-5-carboxylate synthase",
  "gene_symbol": "ALDH18A1",
  "term_label": "Unknown biological process",
  "gene": "UniProtKB:P54886",
  "term_id": "UNKNOWN:0002"
}